{
  "gene": "UniProtKB:P22307",
  "gene_symbol": "SCP2",
  "term_label": "Unknown molecular function",
  "gene_name": "Sterol carrier protein 2",
  "term_id": "UNKNOWN:0001"
}